chloride channel complex [GO:0034707] (cellular component) Relationships: is a type of GO:0034702 Definition: An ion channel complex through which chloride ions pass. Sources: GOC:mah Subtypes: GO:0016935, histamine-gated chloride channel complex [GO:0019183]